{
  "gene": "UniProtKB:Q6ZRI0",
  "term_label": "Unknown biological process",
  "gene_symbol": "OTOG",
  "term_id": "UNKNOWN:0002",
  "gene_name": "Otogelin"
}